{
  "term_id": "GO:0000977",
  "gene_symbol": "ZNF343",
  "gene": "UniProtKB:Q6P1L6",
  "term_label": "RNA polymerase II transcription regulatory region sequence-specific DNA binding",
  "gene_name": "Zinc finger protein 343"
}